mitotic anaphase [GO:0000090] (biological process) Definition: The cell cycle phase during which chromosomes separate and migrate towards the poles of the spindle the as part of a mitotic cell cycle. Sources: GOC:mtg_cell_cycle Note: Note that this term should not be used for direct annotation. If you are trying to make an annotation to x phase, it is likely that the correct annotation is 'regulation of x/y phase transition' or to a process which occurs during the reported phase (i.e mitotic DNA replication for mitotic S-phase). To capture the phase when a specific location or process is observed, the phase term can be used in an annotation extension (PMID:24885854) applied to a cellular component term (with the relation exists_during) or a biological process term (with the relation happens_during). Relationships: is a type of GO:0051322; is part of mitotic M phase [GO:0000087] Subtypes: mitotic anaphase A [GO:0000091], mitotic anaphase B [GO:0000092]